{
  "gene": "UniProtKB:Q7RTN6",
  "term_label": "serine/threonine protein kinase complex",
  "gene_name": "STE20-related kinase adapter protein alpha",
  "term_id": "GO:1902554",
  "gene_symbol": "STRADA"
}